{
  "gene_name": "Probable ATP-dependent RNA helicase DDX47",
  "gene": "UniProtKB:Q9H0S4",
  "gene_symbol": "DDX47",
  "term_id": "UNKNOWN:0001",
  "term_label": "Unknown molecular function"
}